{
  "term_id": "GO:0005886",
  "gene": "UniProtKB:Q7Z699",
  "gene_name": "Sprouty-related, EVH1 domain-containing protein 1",
  "term_label": "plasma membrane",
  "gene_symbol": "SPRED1"
}